{
  "term_id": "GO:0000814",
  "term_label": "ESCRT II complex",
  "gene_name": "Vacuolar-sorting protein SNF8",
  "gene": "UniProtKB:Q96H20",
  "gene_symbol": "SNF8"
}